positive regulation of 7-methylguanosine mRNA capping [GO:0160199] (BP) Relationships: is a type of positive regulation of mRNA processing [GO:0050685]; positively regulates 7-methylguanosine mRNA capping [GO:0006370] References: PMID:19328067 Definition: Any process that activates or increases the frequency, rate or extent of 7-methylguanosine mRNA capping.